{
  "term_id": "GO:0043409",
  "term_label": "negative regulation of MAPK cascade",
  "gene_symbol": "STYXL2",
  "gene_name": "Serine_threonine_tyrosine-interacting-like protein 2",
  "gene": "UniProtKB:Q5VZP5"
}